{
  "term_id": "UNKNOWN:0002",
  "term_label": "Unknown biological process",
  "gene_symbol": "KRTAP9-2",
  "gene_name": "Keratin-associated protein 9-2",
  "gene": "UniProtKB:Q9BYQ4"
}